{
  "gene": "UniProtKB:Q9P031",
  "gene_name": "Thyroid transcription factor 1-associated protein 26",
  "term_id": "GO:0005634",
  "term_label": "nucleus",
  "gene_symbol": "CCDC59"
}